{
  "term_label": "actin binding",
  "gene_symbol": "SYNPO2L",
  "gene": "UniProtKB:Q9H987",
  "term_id": "GO:0003779",
  "gene_name": "Synaptopodin 2-like protein"
}